{
  "term_label": "defense response to bacterium",
  "gene_symbol": "MPEG1",
  "gene": "UniProtKB:Q2M385",
  "gene_name": "Macrophage-expressed gene 1 protein",
  "term_id": "GO:0042742"
}